{
  "term_label": "positive regulation of protein catabolic process",
  "gene_name": "Ankyrin repeat and SOCS box protein 5",
  "term_id": "GO:0045732",
  "gene_symbol": "ASB5",
  "gene": "UniProtKB:Q8WWX0"
}